DNA damage response [GO:0006974] (biological process) Definition: Any process that results in a change in state or activity of a cell (in terms of movement, secretion, enzyme production, gene expression, etc.) as a result of a stimulus indicating damage to its DNA from environmental insults or errors during metabolism. Also known as: response to DNA damage stimulus, cellular DNA damage response, cellular response to DNA damage stimulus, response to genotoxic stress Sources: GOC:go_curators Subtypes: GO:0006281, DNA damage tolerance [GO:0006301], GO:0008630, SOS response [GO:0009432], signal transduction in response to DNA damage [GO:0042770], telomere maintenance in response to DNA damage [GO:0043247] Relationships: is a type of cellular response to stress [GO:0033554]